{
  "gene_name": "Dual specificity protein phosphatase 3",
  "term_label": "positive regulation of mitotic cell cycle",
  "gene": "UniProtKB:P51452",
  "gene_symbol": "DUSP3",
  "term_id": "GO:0045931"
}